{
  "gene_name": "Reticulon-2",
  "term_label": "endoplasmic reticulum tubular network membrane organization",
  "gene": "UniProtKB:O75298",
  "gene_symbol": "RTN2",
  "term_id": "GO:1990809"
}